{
  "gene_symbol": "GPR107",
  "term_label": "clathrin-dependent endocytosis",
  "gene": "UniProtKB:Q5VW38",
  "term_id": "GO:0072583",
  "gene_name": "Protein GPR107"
}